{
  "gene": "UniProtKB:O75791",
  "gene_name": "GRB2-related adapter protein 2",
  "gene_symbol": "GRAP2",
  "term_label": "nucleoplasm",
  "term_id": "GO:0005654"
}